diphosphoinositol tetrakisphosphate kinase activity [GO:0052839] (molecular function) Relationships: is_a phosphotransferase activity, alcohol group as acceptor [GO:0016773]; is a type of inositol phosphate kinase activity [GO:0180030] References: PMID:10827188, PMID:11502751, PMID:18355727 Also known as: PP-IP4 kinase activity, inositol diphosphate tetrakisphosphate kinase activity Definition: Catalysis of the reaction: ATP + diphospho-1D-myo-inositol tetrakisphosphate = ADP + bis(diphospho)-1D-myo-inositol trisphosphate.